{
  "gene_symbol": "SYTL4",
  "gene_name": "Synaptotagmin-like protein 4",
  "gene": "UniProtKB:Q96C24",
  "term_id": "GO:0070382",
  "term_label": "exocytic vesicle"
}